{
  "gene_name": "Tyrosine 3-monooxygenase",
  "gene": "UniProtKB:P07101",
  "gene_symbol": "TH",
  "term_label": "cytoplasm",
  "term_id": "GO:0005737"
}